signal transduction involved in cellular response to ammonium ion [GO:1903831] (biological process) Definition: Any signal transduction that is involved in cellular response to ammonium ion. Also known as: signaling cascade involved in cellular response to ammonium ion, signalling cascade involved in cellular response to ammonium ion, signaling pathway involved in cellular response to ammonium ion, signalling pathway involved in cellular response to ammonium ion Relationships: is a type of signal transduction [GO:0007165]; is part of cellular response to ammonium ion [GO:0071242] References: PMID:16297994 Sources: GOC:TermGenie, GO_REF:0000060